{
  "term_id": "UNKNOWN:0003",
  "gene": "UniProtKB:Q9H293",
  "gene_name": "Interleukin-25",
  "term_label": "Unknown cellular component",
  "gene_symbol": "IL25"
}